{
  "term_label": "endoplasmic reticulum",
  "gene_name": "N-terminal EF-hand calcium-binding protein 3",
  "gene": "UniProtKB:Q96P71",
  "gene_symbol": "NECAB3",
  "term_id": "GO:0005783"
}